{
  "gene_name": "Connector enhancer of kinase suppressor of ras 2",
  "term_id": "GO:0005886",
  "gene": "UniProtKB:Q8WXI2",
  "term_label": "plasma membrane",
  "gene_symbol": "CNKSR2"
}